template-free RNA nucleotidyltransferase [GO:0098680] (molecular function) Definition: Catalysis of the reaction: nucleoside triphosphate + RNA(n) = diphosphate + RNA(n+1); the addition of a terminal nucleotide to an RNA molecule in the absence of a nucleic acid template. Relationships: is a type of GO:0016779; is a type of GO:0140098 References: PMID:15994230 Sources: GOC:BHF, GOC:BHF_telomere, GOC:dos, GOC:nc